{
  "gene_symbol": "ANKRD30BL",
  "term_label": "Unknown molecular function",
  "gene": "UniProtKB:A7E2S9",
  "term_id": "UNKNOWN:0001",
  "gene_name": "Putative ankyrin repeat domain-containing protein 30B-like"
}